{
  "term_label": "delayed rectifier potassium channel activity",
  "gene_name": "Potassium voltage-gated channel subfamily A member 10",
  "gene_symbol": "KCNA10",
  "gene": "UniProtKB:Q16322",
  "term_id": "GO:0005251"
}